{
  "gene_name": "cAMP-dependent protein kinase inhibitor alpha",
  "gene_symbol": "PKIA",
  "gene": "UniProtKB:P61925",
  "term_id": "UNKNOWN:0002",
  "term_label": "Unknown biological process"
}